maternal process involved in parturition [GO:0060137] (biological process) Relationships: is a type of multicellular organismal reproductive process [GO:0048609]; BFO_0000050 parturition [GO:0007567] Definition: A reproductive process occurring in the mother that results in birth. Sources: GOC:dph Regulation: regulated by regulation of maternal process involved in parturition [GO:1904301]; negatively regulated by negative regulation of maternal process involved in parturition [GO:1904302]; positively regulated by positive regulation of maternal process involved in parturition [GO:1904303]